{
  "term_id": "GO:0005737",
  "gene": "UniProtKB:Q96J92",
  "gene_name": "Serine_threonine-protein kinase WNK4",
  "term_label": "cytoplasm",
  "gene_symbol": "WNK4"
}